solute:monoatomic cation symporter activity [GO:0015294] (molecular function) Also known as: solute:cation symporter activity Sources: GOC:ai Subtypes: carbohydrate:monoatomic cation symporter activity [GO:0005402], amino acid:monoatomic cation symporter activity [GO:0005416], GO:0015295, monoatomic anion:monoatomic cation symporter activity [GO:0015296], GO:0015306, solute:sodium symporter activity [GO:0015370], GO:0015391, GO:0015539, acetate:monoatomic cation symporter activity [GO:0043893], GO:0140410 Definition: Enables the transfer of a solute or solutes from one side of a membrane to the other according to the reaction: solute(out) + cation(out) = solute(in) + cation(in). Relationships: is a type of GO:0008324; is a type of symporter activity [GO:0015293]